{
  "gene_symbol": "CITED1",
  "gene": "UniProtKB:Q99966",
  "term_id": "GO:0030318",
  "term_label": "melanocyte differentiation",
  "gene_name": "Cbp_p300-interacting transactivator 1"
}